{
  "gene": "UniProtKB:Q4G0J3",
  "gene_symbol": "LARP7",
  "gene_name": "La-related protein 7",
  "term_label": "Unknown biological process",
  "term_id": "UNKNOWN:0002"
}